{
  "term_id": "GO:0005689",
  "gene": "UniProtKB:Q16560",
  "gene_name": "U11_U12 small nuclear ribonucleoprotein 35 kDa protein",
  "gene_symbol": "SNRNP35",
  "term_label": "U12-type spliceosomal complex"
}